{
  "term_id": "GO:0045944",
  "gene_name": "Basic helix-loop-helix domain-containing protein USF3",
  "gene": "UniProtKB:Q68DE3",
  "gene_symbol": "USF3",
  "term_label": "positive regulation of transcription by RNA polymerase II"
}